{
  "gene": "UniProtKB:Q14168",
  "term_label": "plasma membrane",
  "term_id": "GO:0005886",
  "gene_symbol": "MPP2",
  "gene_name": "MAGUK p55 subfamily member 2"
}